{
  "gene_symbol": "SYF2",
  "term_label": "post-mRNA release spliceosomal complex",
  "gene": "UniProtKB:O95926",
  "term_id": "GO:0071014",
  "gene_name": "Pre-mRNA-splicing factor SYF2"
}